venom-mediated vasoconstriction [GO:0044499] (biological process) References: PMID:19837656 Sources: GOC:fj Also known as: envenomation resulting in positive regulation of blood pressure in another organism, envenomation resulting in positive regulation of blood pressure in other organism, venom-mediated increase in blood pressure in another organism Definition: A process in which an organism initiates, promotes, or enhances the narrowing (constriction) of blood vessels by small muscles in their walls in another organism via the action of a venom, concomittantly increasing blood pressure in the bitten/stung organism. Relationships: is a type of venom-mediated perturbation of blood circulation [GO:0140134]